{
  "gene_symbol": "PSIP1",
  "gene_name": "PC4 and SFRS1-interacting protein",
  "gene": "UniProtKB:O75475",
  "term_label": "nucleus",
  "term_id": "GO:0005634"
}